{
  "term_id": "GO:0005669",
  "gene_symbol": "TAF4B",
  "term_label": "transcription factor TFIID complex",
  "gene": "UniProtKB:Q92750",
  "gene_name": "Transcription initiation factor TFIID subunit 4B"
}